{
  "gene_name": "IQ and AAA domain-containing protein 1-like",
  "term_label": "nucleus",
  "term_id": "GO:0005634",
  "gene_symbol": "IQCA1L",
  "gene": "UniProtKB:A6NCM1"
}